{
  "gene_symbol": "MTCL1",
  "term_label": "apicolateral plasma membrane",
  "gene_name": "Microtubule cross-linking factor 1",
  "term_id": "GO:0016327",
  "gene": "UniProtKB:Q9Y4B5"
}